{
  "term_id": "GO:0048259",
  "gene_symbol": "ANKRD13B",
  "gene_name": "Ankyrin repeat domain-containing protein 13B",
  "term_label": "regulation of receptor-mediated endocytosis",
  "gene": "UniProtKB:Q86YJ7"
}